{
  "gene_symbol": "NSUN5",
  "term_id": "GO:0070475",
  "term_label": "rRNA base methylation",
  "gene": "UniProtKB:Q96P11",
  "gene_name": "28S rRNA (cytosine-C(5))-methyltransferase"
}